{
  "gene_symbol": "LTC4S",
  "term_id": "GO:0004364",
  "gene_name": "Leukotriene C4 synthase",
  "gene": "UniProtKB:Q16873",
  "term_label": "glutathione transferase activity"
}